{
  "gene": "UniProtKB:Q96PL1",
  "gene_name": "Secretoglobin family 3A member 2",
  "term_id": "UNKNOWN:0001",
  "gene_symbol": "SCGB3A2",
  "term_label": "Unknown molecular function"
}